{
  "term_label": "Unknown cellular component",
  "term_id": "UNKNOWN:0003",
  "gene_name": "Uncharacterized protein encoded by LINC01587",
  "gene": "UniProtKB:Q99440",
  "gene_symbol": "LINC01587"
}